muscle hypertrophy [GO:0014896] (biological process) Relationships: is a type of GO:0003012 Sources: GOC:mtg_muscle Definition: The muscle system process that results in enlargement or overgrowth of all or part of a muscle organ due to an increase in the size of its muscle cells. Physiological hypertrophy is a normal process during development (it stops in cardiac muscle after adolescence) and can also be brought on in response to demand. In athletes cardiac and skeletal muscles undergo hypertrophy stimulated by increasing muscle activity on exercise. Smooth muscle cells in the uterus undergo hypertrophy during pregnancy. Subtypes: physiological muscle hypertrophy [GO:0003298], muscle hypertrophy in response to stress [GO:0003299], smooth muscle hypertrophy [GO:0014895], striated muscle hypertrophy [GO:0014897] Regulation: negatively regulated by GO:0014741; positively regulated by positive regulation of muscle hypertrophy [GO:0014742]; regulated by GO:0014743